histone H3K4 demethylase activity [GO:0032453] (molecular function) Sources: GOC:mah Relationships: is a type of histone H3 demethylase activity [GO:0141052] Also known as: histone H3-K4 demethylase activity, histone H3-methyl-lysine-4 demethylase activity, histone demethylase activity (H3-K4 specific), histone demethylase activity (H3K4-specific) Subtypes: histone H3K4me/H3K4me2/H3K4me3 demethylase activity [GO:0034647], FAD-dependent H3K4me/H3K4me3 demethylase activity [GO:0140682] Definition: Catalysis of the removal of a methyl group from a modified lysine residue at position 4 of the histone H3 protein. Note: Comment: Note that the residue position corresponds to the canonical human H3 histone (UniProtKB:P84243); this residue is conserved across all eukaryotes. Residue 1 is the first residue following removal of the initiating Methionine (Met). Note that each histone is encoded by multiple genes, and sequences may vary across different genes within an organism.